regulation of myeloid cell differentiation [GO:0045637] (biological process) Subtypes: GO:0002761, negative regulation of myeloid cell differentiation [GO:0045638], positive regulation of myeloid cell differentiation [GO:0045639], GO:0045646, regulation of megakaryocyte differentiation [GO:0045652], regulation of platelet formation [GO:1905219] Relationships: is a type of regulation of hemopoiesis [GO:1903706]; regulates GO:0030099 Definition: Any process that modulates the frequency, rate or extent of myeloid cell differentiation. Sources: GOC:go_curators